negative regulation of t-SNARE clustering [GO:1904033] (biological process) Definition: Any process that stops, prevents or reduces the frequency, rate or extent of t-SNARE clustering. Also known as: down regulation of t-SNARE clustering, down-regulation of t-SNARE clustering, downregulation of t-SNARE clustering, inhibition of t-SNARE clustering Relationships: is a type of regulation of t-SNARE clustering [GO:1904032]; is a type of negative regulation of protein localization to membrane [GO:1905476]; negatively regulates GO:1990656 References: PMID:22528485 Sources: GOC:TermGenie, GO_REF:0000058